{
  "gene_symbol": "STC1",
  "gene": "UniProtKB:P52823",
  "gene_name": "Stanniocalcin-1",
  "term_label": "intracellular calcium ion homeostasis",
  "term_id": "GO:0006874"
}